{
  "gene_symbol": "ZNF587",
  "term_id": "GO:0005634",
  "gene": "UniProtKB:Q96SQ5",
  "term_label": "nucleus",
  "gene_name": "Zinc finger protein 587"
}